{
  "gene_symbol": "CASP7",
  "gene_name": "Caspase-7",
  "gene": "UniProtKB:P55210",
  "term_id": "GO:0004197",
  "term_label": "cysteine-type endopeptidase activity"
}